{
  "term_id": "GO:0004888",
  "term_label": "transmembrane signaling receptor activity",
  "gene_symbol": "FCRL3",
  "gene": "UniProtKB:Q96P31",
  "gene_name": "Fc receptor-like protein 3"
}